{
  "term_label": "chemical synaptic transmission",
  "gene_name": "Muscarinic acetylcholine receptor M5",
  "term_id": "GO:0007268",
  "gene": "UniProtKB:P08912",
  "gene_symbol": "CHRM5"
}